lymphoid lineage cell migration into thymus [GO:0097535] (biological process) References: PMID:22342843 Sources: GOC:cvs Also known as: lymphoid lineage restricted progenitor cell migration into thymus Definition: The movement of a lymphoid lineage cell (also called a lymphoid lineage restricted progenitor cell) into the thymus. Lymphoid lineage cells enter and exit the thymus several times as part of this process. Relationships: is a type of GO:0097534 Subtypes: GO:1902550